{
  "gene_name": "tRNA (adenine(58)-N(1))-methyltransferase non-catalytic subunit TRM6",
  "term_label": "tRNA (m1A) methyltransferase complex",
  "gene": "UniProtKB:Q9UJA5",
  "term_id": "GO:0031515",
  "gene_symbol": "TRMT6"
}